fosmidomycin transport [GO:0042894] (biological process) Relationships: is a type of amide transport [GO:0042886] References: PMID:12543685 Sources: GOC:jl Definition: The directed movement of fosmidomycin, a phosphonic acid derivative with potent activity against Gram-negative organisms, into, out of or within a cell, or between cells, by means of some agent such as a transporter or pore.